{
  "term_label": "Rho protein signal transduction",
  "term_id": "GO:0007266",
  "gene_symbol": "CDC42EP1",
  "gene_name": "Cdc42 effector protein 1",
  "gene": "UniProtKB:Q00587"
}